{
  "gene_symbol": "CXXC1",
  "gene": "UniProtKB:Q9P0U4",
  "term_label": "Unknown molecular function",
  "gene_name": "CXXC-type zinc finger protein 1",
  "term_id": "UNKNOWN:0001"
}